glycolytic process through fructose-1-phosphate [GO:0061625] (biological process) Definition: The chemical reactions and pathways resulting in the breakdown of fructose into pyruvate through a fructose-1-phosphate intermediate, with the concomitant production of ATP and NADH. Sources: GOC:dph, ISBN:0201090910 Relationships: is a type of fructose catabolic process [GO:0006001]; is a type of glycolytic process [GO:0006096]; has part GO:0004807; has part fructose catabolic process to hydroxyacetone phosphate and glyceraldehyde-3-phosphate [GO:0061624]